{
  "term_label": "CCR chemokine receptor binding",
  "gene_symbol": "CCL3L1",
  "term_id": "GO:0048020",
  "gene_name": "C-C motif chemokine 3-like 1",
  "gene": "UniProtKB:P16619"
}